{
  "gene_name": "Olfactory receptor 7E24",
  "term_label": "plasma membrane",
  "gene": "UniProtKB:Q6IFN5",
  "term_id": "GO:0005886",
  "gene_symbol": "OR7E24"
}